{
  "gene": "UniProtKB:Q9HBH0",
  "gene_symbol": "RHOF",
  "gene_name": "Rho-related GTP-binding protein RhoF",
  "term_id": "GO:0032956",
  "term_label": "regulation of actin cytoskeleton organization"
}